{
  "gene_symbol": "MLLT1",
  "term_id": "GO:0003682",
  "gene_name": "Protein ENL",
  "term_label": "chromatin binding",
  "gene": "UniProtKB:Q03111"
}